glycine biosynthetic process, by transamination of glyoxylate [GO:0019265] (biological process) Sources: GOC:go_curators Definition: The chemical reactions and pathways resulting in the formation of glycine by the transamination of glyoxylate. Relationships: is a type of glycine biosynthetic process [GO:0006545] Also known as: glycine anabolism, by transamination of glyoxylate, glycine formation, by transamination of glyoxylate, glycine synthesis, by transamination of glyoxylate